{
  "gene_name": "Prepronociceptin",
  "gene_symbol": "PNOC",
  "gene": "UniProtKB:Q13519",
  "term_label": "chemical synaptic transmission",
  "term_id": "GO:0007268"
}